{
  "term_id": "GO:0030172",
  "term_label": "troponin C binding",
  "gene": "UniProtKB:P45378",
  "gene_symbol": "TNNT3",
  "gene_name": "Troponin T, fast skeletal muscle"
}